{
  "term_label": "cytoplasm",
  "term_id": "GO:0005737",
  "gene_name": "NK-tumor recognition protein",
  "gene": "UniProtKB:P30414",
  "gene_symbol": "NKTR"
}